{
  "term_id": "UNKNOWN:0002",
  "term_label": "Unknown biological process",
  "gene_name": "Ankyrin repeat and SAM domain-containing protein 6",
  "gene": "UniProtKB:Q68DC2",
  "gene_symbol": "ANKS6"
}